protein octanoylation [GO:0018190] (biological process) Definition: The modification of a protein amino acid by formation of an ester or amide with octanoic acid. Sources: GOC:jsg Also known as: protein amino acid octanoylation Relationships: is a type of protein lipidation [GO:0006497]; is a type of protein acylation [GO:0043543] Subtypes: GO:0018191